nucleolar chromatin organization [GO:1990700] (biological process) Relationships: is a type of GO:0006325; is part of chromatin organization [GO:0006325]; is part of GO:0007000 References: PMID:18362178 Also known as: establishment or maintenance of nucleolar chromatin architecture, nucleolar chromatin organisation Definition: Any process that results in the specification, formation or maintenance of the physical structure of nucleolar chromatin.